extrinsic component of mycolate outer membrane [GO:0036420] (cellular component) Relationships: is a type of extrinsic component of cell outer membrane [GO:0031244]; is part of mycolate outer membrane [GO:0036407] Definition: The component of mycolate outer membrane consisting of gene products and protein complexes that are loosely bound to one of its surfaces, but not integrated into the hydrophobic region. Also known as: extrinsic to MOM, extrinsic to mycomembrane, extrinsic to mycolate outer membrane Subtypes: extrinsic component of external side of mycolate outer membrane [GO:0036421] Sources: GOC:dos, GOC:md